7-cyano-7-deazaguanine biosynthetic process [GO:0097288] (biological process) Also known as: 7-cyano-7-deazaguanine anabolism, 7-cyano-7-deazaguanine biosynthesis, 7-cyano-7-deazaguanine formation, 7-cyano-7-deazaguanine synthesis Relationships: is a type of nitrile biosynthetic process [GO:0080028]; is a type of 7-cyano-7-deazaguanine metabolic process [GO:0097287] References: PMID:364423 Sources: GOC:yaf Definition: The chemical reactions and pathways resulting in the formation of the Q nucleoside precursor 7-cyano-7-deazaguanine, also known as 2-amino-4-oxo-4,7-dihydro-3H-pyrrolo[2,3-d]pyrimidine-5-carbonitrile or preQo.